{
  "gene_symbol": "EXOC4",
  "term_label": "Golgi to plasma membrane transport",
  "gene": "UniProtKB:Q96A65",
  "gene_name": "Exocyst complex component 4",
  "term_id": "GO:0006893"
}